{
  "gene": "UniProtKB:P07900",
  "term_label": "cytosol",
  "gene_name": "Heat shock protein HSP 90-alpha",
  "term_id": "GO:0005829",
  "gene_symbol": "HSP90AA1"
}